{
  "gene": "UniProtKB:Q6UWR7",
  "term_id": "GO:0008889",
  "gene_symbol": "ENPP6",
  "gene_name": "Glycerophosphocholine cholinephosphodiesterase ENPP6",
  "term_label": "glycerophosphodiester phosphodiesterase activity"
}